{
  "gene_symbol": "MYOC",
  "term_label": "Unknown molecular function",
  "term_id": "UNKNOWN:0001",
  "gene": "UniProtKB:Q99972",
  "gene_name": "Myocilin"
}